{
  "term_label": "Unknown cellular component",
  "gene_symbol": "RNF220",
  "term_id": "UNKNOWN:0003",
  "gene": "UniProtKB:Q5VTB9",
  "gene_name": "E3 ubiquitin-protein ligase RNF220"
}